{
  "term_label": "axon",
  "term_id": "GO:0030424",
  "gene_name": "Potassium voltage-gated channel subfamily A member 3",
  "gene": "UniProtKB:P22001",
  "gene_symbol": "KCNA3"
}